{
  "term_id": "GO:0008296",
  "gene_name": "DNA polymerase delta catalytic subunit",
  "gene_symbol": "POLD1",
  "gene": "UniProtKB:P28340",
  "term_label": "3'-5'-DNA exonuclease activity"
}